{
  "gene_symbol": "MTRNR2L12",
  "gene_name": "Humanin-like 12",
  "term_label": "Unknown biological process",
  "term_id": "UNKNOWN:0002",
  "gene": "UniProtKB:P0DMP1"
}